regulation of phosphorus utilization [GO:0006795] (biological process) Sources: GOC:go_curators Relationships: is a type of GO:0051174; regulates phosphorus utilization [GO:0006794] Definition: Any process that modulates the frequency, rate or extent of phosphorus utilization. Subtypes: negative regulation of phosphorus utilization [GO:0045942], positive regulation of phosphorus utilization [GO:0045949]